{
  "term_label": "Unknown molecular function",
  "gene_symbol": "TRBJ2-2",
  "term_id": "UNKNOWN:0001",
  "gene_name": "T cell receptor beta joining 2-2",
  "gene": "UniProtKB:A0A0A0MT94"
}